{
  "term_id": "GO:0016540",
  "gene_name": "Myelin regulatory factor-like protein",
  "gene_symbol": "MYRFL",
  "gene": "UniProtKB:Q96LU7",
  "term_label": "protein autoprocessing"
}